embryonic digestive tract morphogenesis [GO:0048557] (biological process) Definition: The process in which the anatomical structures of the digestive tract are generated and organized during embryonic development. The digestive tract is the anatomical structure through which food passes and is processed. Relationships: is a type of embryonic organ morphogenesis [GO:0048562]; is part of digestive tract morphogenesis [GO:0048546]; is part of embryonic digestive tract development [GO:0048566] Sources: GOC:go_curators Also known as: embryonic gut morphogenesis